{
  "gene_name": "Dynein regulatory complex protein 10",
  "gene_symbol": "IQCD",
  "gene": "UniProtKB:Q96DY2",
  "term_id": "UNKNOWN:0003",
  "term_label": "Unknown cellular component"
}